vascular endothelial growth factor signaling pathway [GO:0038084] (biological process) Also known as: VEGF signaling, VEGF-activated signaling pathway, vascular endothelial growth factor signalling pathway Definition: The series of molecular signals initiated by vascular endothelial growth factor (VEGF) binding its receptor on the surface of the target cell, and ending with the regulation of a downstream cellular process, e.g. transcription. Subtypes: VEGF-activated platelet-derived growth factor receptor signaling pathway [GO:0038086], positive regulation of cell migration by vascular endothelial growth factor signaling pathway [GO:0038089], VEGF-activated neuropilin signaling pathway [GO:0038190] Relationships: is_a cell surface receptor protein tyrosine kinase signaling pathway [GO:0007169]; is part of cellular response to vascular endothelial growth factor stimulus [GO:0035924] Regulation: regulated by GO:1900746; negatively regulated by GO:1900747; positively regulated by positive regulation of vascular endothelial growth factor signaling pathway [GO:1900748] Note: In GO, a gene product with 'vascular endothelial growth factor-activated receptor activity ; GO:0005021' necessarily binds VEGF to transduce a signal. To represent cross-talk between ligands and receptors, signaling pathways in GO are starting to be named after the receptor and/or the signal. GO:0038084 is for annotation of any pathway in which the ligand VEGF binds and activates any cell surface receptor (VEGFR, PDGFR etc.). For annotation of signaling pathways where a VEGFR binds one of its physiological ligands (VEGF or an alternative growth factor), consider 'vascular endothelial growth factor receptor signaling pathway ; GO:0048010'. References: PMID:17470632 Sources: GOC:signaling